{
  "term_label": "intracellular potassium ion homeostasis",
  "gene_symbol": "ATP1B2",
  "gene_name": "Sodium_potassium-transporting ATPase subunit beta-2",
  "term_id": "GO:0030007",
  "gene": "UniProtKB:P14415"
}